negative regulation of leukocyte mediated immunity [GO:0002704] (biological process) Also known as: down regulation of leukocyte mediated immunity, down-regulation of leukocyte mediated immunity, downregulation of leukocyte mediated immunity, negative regulation of immune cell mediated immunity, negative regulation of leucocyte mediated immunity, inhibition of leukocyte mediated immunity Sources: GOC:add Subtypes: negative regulation of leukocyte mediated cytotoxicity [GO:0001911], GO:0002707, negative regulation of dendritic cell cytokine production [GO:0002731], negative regulation of myeloid leukocyte mediated immunity [GO:0002887] Definition: Any process that stops, prevents, or reduces the frequency, rate, or extent of leukocyte mediated immunity. Relationships: is_a negative regulation of immune effector process [GO:0002698]; is a type of GO:0002703; negatively regulates leukocyte mediated immunity [GO:0002443]